{
  "gene_symbol": "PIAS3",
  "gene": "UniProtKB:Q9Y6X2",
  "term_id": "GO:0061665",
  "term_label": "SUMO ligase activity",
  "gene_name": "E3 SUMO-protein ligase PIAS3"
}